{
  "gene_symbol": "SMIM27",
  "term_label": "Unknown molecular function",
  "gene": "UniProtKB:A0A1B0GUW7",
  "gene_name": "Small integral membrane protein 27",
  "term_id": "UNKNOWN:0001"
}